regulation of glycerol transport [GO:0090371] (biological process) Relationships: is a type of regulation of transmembrane transport [GO:0034762]; regulates glycerol transmembrane transport [GO:0015793] Definition: Any process that modulates the rate, frequency, or extent of the directed movement of glycerol into, out of or within a cell, or between cells, by means of some agent such as a transporter or pore. Sources: GOC:dph, GOC:jh, GOC:tb Subtypes: positive regulation of glycerol transport [GO:0090372], negative regulation of glycerol transport [GO:0090373]